regulation of hyaluranon cable assembly [GO:1900104] (biological process) Also known as: regulation of HA cable assembly Definition: Any process that modulates the frequency, rate or extent of hyaluranon cable assembly. Sources: GOC:TermGenie, GOC:yaf Subtypes: negative regulation of hyaluranon cable assembly [GO:1900105], GO:1900106 Relationships: is_a regulation of cellular component biogenesis [GO:0044087]; is a type of regulation of cellular component organization [GO:0051128]; regulates GO:0036118